{
  "gene_name": "Guanine nucleotide-binding protein subunit alpha-15",
  "term_id": "UNKNOWN:0002",
  "term_label": "Unknown biological process",
  "gene": "UniProtKB:P30679",
  "gene_symbol": "GNA15"
}